{
  "term_id": "GO:0005789",
  "term_label": "endoplasmic reticulum membrane",
  "gene_name": "Stimulator of interferon genes protein",
  "gene_symbol": "STING1",
  "gene": "UniProtKB:Q86WV6"
}